{
  "gene_symbol": "LDHA",
  "gene": "UniProtKB:P00338",
  "term_id": "GO:0006089",
  "gene_name": "L-lactate dehydrogenase A chain",
  "term_label": "lactate metabolic process"
}